positive regulation of nephron tubule epithelial cell differentiation [GO:2000768] (biological process) Relationships: is a type of regulation of nephron tubule epithelial cell differentiation [GO:0072182]; is a type of GO:2000698; positively regulates nephron tubule epithelial cell differentiation [GO:0072160] Sources: GOC:obol Definition: Any process that activates or increases the frequency, rate or extent of nephron tubule epithelial cell differentiation.